protein secretion by the type V secretion system [GO:0046819] (biological process) Also known as: autotransporter system, protein secretion by the autotransporter system, protein secretion by the type V protein secretion system, type V protein secretion system Relationships: is a type of GO:0009306; is a type of protein transport across the cell outer membrane [GO:0098776] Sources: GOC:pamgo_curators Definition: The process in which proteins mediate their own secretion across the outer membrane through a beta-barrel pore structure formed by the C-terminal domain of the protein precursor. Following passage across the outer membrane, the mature protein is released from the pore by an autocatalytic activity. Proteins secreted by the Type V system are first translocated across the plasma membrane by the Sec pathway.